peptide dopaminyltransferase activity [GO:0120296] (molecular function) Subtypes: GO:0120297 References: PMID:22858378, PMID:32273471 Sources: GOC:sp Definition: Catalysis of the reaction: dopamine + L-glutaminyl-[protein] = 5-dopaminyl-L-glutamyl-[protein] + NH4(+). Relationships: is a type of N-acyltransferase activity [GO:0016410]